{
  "gene_name": "Adenosine 3'-phospho 5'-phosphosulfate transporter 2",
  "gene": "UniProtKB:Q9H1N7",
  "term_id": "GO:0000139",
  "term_label": "Golgi membrane",
  "gene_symbol": "SLC35B3"
}